{
  "term_id": "GO:0033209",
  "gene_name": "TNF receptor-associated factor 2",
  "term_label": "tumor necrosis factor-mediated signaling pathway",
  "gene_symbol": "TRAF2",
  "gene": "UniProtKB:Q12933"
}